{
  "term_id": "GO:0005615",
  "gene_symbol": "TCN1",
  "gene_name": "Transcobalamin-1",
  "gene": "UniProtKB:P20061",
  "term_label": "extracellular space"
}